{
  "term_id": "GO:0008284",
  "gene": "UniProtKB:Q9HC73",
  "gene_name": "Cytokine receptor-like factor 2",
  "term_label": "positive regulation of cell population proliferation",
  "gene_symbol": "CRLF2"
}